cellular response to nitrogen starvation [GO:0006995] (biological process) Relationships: is a type of GO:0009267; is a type of GO:0043562 Regulation: negatively regulated by negative regulation of cellular response to nitrogen starvation [GO:0010516] Subtypes: induction of conjugation upon nitrogen starvation [GO:0031142] Sources: GOC:jl Definition: Any process that results in a change in state or activity of a cell (in terms of movement, secretion, enzyme production, gene expression, etc.) as a result of deprivation of nitrogen.